{
  "term_id": "GO:0045944",
  "gene": "UniProtKB:Q10586",
  "gene_symbol": "DBP",
  "term_label": "positive regulation of transcription by RNA polymerase II",
  "gene_name": "D site-binding protein"
}